positive regulation of glucose mediated signaling pathway [GO:1902661] (biological process) Definition: Any process that activates or increases the frequency, rate or extent of glucose mediated signaling pathway. Relationships: is a type of positive regulation of signal transduction [GO:0009967]; is a type of GO:1902659; positively regulates glucose mediated signaling pathway [GO:0010255] References: PMID:24277933 Sources: GOC:TermGenie, GOC:di, GO_REF:0000058 Also known as: positive regulation of glucose mediated signalling, up regulation of glucose mediated signaling pathway, up regulation of glucose mediated signalling, up-regulation of glucose mediated signaling pathway, up-regulation of glucose mediated signalling, upregulation of glucose mediated signaling pathway, upregulation of glucose mediated signalling, activation of glucose mediated signaling pathway, activation of glucose mediated signalling